{
  "term_label": "Unknown cellular component",
  "term_id": "UNKNOWN:0003",
  "gene_symbol": "STAB2",
  "gene": "UniProtKB:Q8WWQ8",
  "gene_name": "Stabilin-2"
}